{
  "term_label": "Unknown molecular function",
  "gene": "UniProtKB:Q3SXP7",
  "gene_symbol": "SHISAL1",
  "term_id": "UNKNOWN:0001",
  "gene_name": "Protein shisa-like-1"
}